{
  "term_label": "Unknown biological process",
  "gene_symbol": "FAM89A",
  "gene": "UniProtKB:Q96GI7",
  "term_id": "UNKNOWN:0002",
  "gene_name": "Protein FAM89A"
}